{
  "term_id": "GO:0071559",
  "gene_name": "Matrix-remodeling-associated protein 5",
  "term_label": "response to transforming growth factor beta",
  "gene": "UniProtKB:Q9NR99",
  "gene_symbol": "MXRA5"
}